{
  "term_id": "UNKNOWN:0003",
  "gene_symbol": "TMEM52B",
  "term_label": "Unknown cellular component",
  "gene_name": "Transmembrane protein 52B",
  "gene": "UniProtKB:Q4KMG9"
}